{
  "term_id": "GO:0004386",
  "gene_symbol": "TDRD9",
  "term_label": "helicase activity",
  "gene_name": "ATP-dependent RNA helicase TDRD9",
  "gene": "UniProtKB:Q8NDG6"
}